{
  "gene": "UniProtKB:Q96PG1",
  "gene_name": "Putative membrane-spanning 4-domains subfamily A member 4E",
  "term_label": "Unknown cellular component",
  "gene_symbol": "MS4A4E",
  "term_id": "UNKNOWN:0003"
}